{
  "term_label": "plasma membrane",
  "gene_symbol": "CD82",
  "gene_name": "CD82 antigen",
  "gene": "UniProtKB:P27701",
  "term_id": "GO:0005886"
}